{
  "gene": "UniProtKB:P24855",
  "gene_name": "Deoxyribonuclease-1",
  "term_label": "DNA binding",
  "gene_symbol": "DNASE1",
  "term_id": "GO:0003677"
}